{
  "term_label": "dendrite",
  "gene": "UniProtKB:P05937",
  "term_id": "GO:0030425",
  "gene_symbol": "CALB1",
  "gene_name": "Calbindin"
}